{
  "term_id": "GO:0005783",
  "term_label": "endoplasmic reticulum",
  "gene": "UniProtKB:Q9Y2G3",
  "gene_symbol": "ATP11B",
  "gene_name": "Phospholipid-transporting ATPase IF"
}